{
  "term_label": "nucleus",
  "gene": "UniProtKB:Q99640",
  "term_id": "GO:0005634",
  "gene_name": "Membrane-associated tyrosine- and threonine-specific cdc2-inhibitory kinase",
  "gene_symbol": "PKMYT1"
}